{
  "gene": "UniProtKB:P39748",
  "term_id": "GO:0030145",
  "term_label": "manganese ion binding",
  "gene_symbol": "FEN1",
  "gene_name": "Flap endonuclease 1"
}